{
  "term_label": "Unknown biological process",
  "gene": "UniProtKB:Q7L3V2",
  "gene_symbol": "RTL10",
  "term_id": "UNKNOWN:0002",
  "gene_name": "Protein Bop"
}